{
  "term_id": "GO:0045202",
  "gene_symbol": "LAMA1",
  "gene_name": "Laminin subunit alpha-1",
  "gene": "UniProtKB:P25391",
  "term_label": "synapse"
}